{
  "term_label": "Unknown biological process",
  "gene": "UniProtKB:A0A0J9YXV3",
  "gene_symbol": "GREP1",
  "term_id": "UNKNOWN:0002",
  "gene_name": "Glycine-rich extracellular protein 1"
}